{
  "term_label": "Unknown molecular function",
  "gene_symbol": "MRPL38",
  "gene_name": "Large ribosomal subunit protein mL38",
  "gene": "UniProtKB:Q96DV4",
  "term_id": "UNKNOWN:0001"
}